negative regulation of blood vessel endothelial cell migration [GO:0043537] (biological process) Definition: Any process that stops, prevents, or reduces the frequency, rate or extent of the migration of the endothelial cells of blood vessels. Sources: GOC:go_curators Also known as: down regulation of blood vessel endothelial cell migration, down-regulation of blood vessel endothelial cell migration, downregulation of blood vessel endothelial cell migration, inhibition of blood vessel endothelial cell migration Relationships: is a type of negative regulation of endothelial cell migration [GO:0010596]; is a type of regulation of blood vessel endothelial cell migration [GO:0043535]; negatively regulates GO:0043534 Subtypes: GO:0090051